{
  "term_label": "ATP-dependent activity, acting on DNA",
  "gene_name": "DNA repair protein RAD51 homolog 4",
  "gene": "UniProtKB:O75771",
  "gene_symbol": "RAD51D",
  "term_id": "GO:0008094"
}